{
  "gene_name": "Vertnin",
  "term_id": "GO:0006357",
  "term_label": "regulation of transcription by RNA polymerase II",
  "gene_symbol": "VRTN",
  "gene": "UniProtKB:Q9H8Y1"
}